{
  "term_label": "DNA-binding transcription factor activity, RNA polymerase II-specific",
  "gene": "UniProtKB:O95936",
  "gene_symbol": "EOMES",
  "term_id": "GO:0000981",
  "gene_name": "Eomesodermin homolog"
}